{
  "gene_name": "Ganglioside-induced differentiation-associated protein 1",
  "gene": "UniProtKB:Q8TB36",
  "term_label": "Unknown molecular function",
  "gene_symbol": "GDAP1",
  "term_id": "UNKNOWN:0001"
}